{
  "term_label": "Unknown cellular component",
  "gene": "UniProtKB:P02751",
  "gene_symbol": "FN1",
  "gene_name": "Fibronectin",
  "term_id": "UNKNOWN:0003"
}